{
  "gene": "UniProtKB:Q9NP73",
  "term_label": "Unknown biological process",
  "gene_name": "Putative bifunctional UDP-N-acetylglucosamine transferase and deubiquitinase ALG13",
  "gene_symbol": "ALG13",
  "term_id": "UNKNOWN:0002"
}